specialized extracellular matrix [GO:0140047] (cellular component) Definition: Species or cell-type specific extracellular matrices that are different from the two main types of extracellular matrices: the interstitial ECM and the basement membrane ECM in metazoa. References: PMID:28955324, PMID:33605520 Also known as: specialized ECM Subtypes: middle lamella [GO:0009519], GO:0033165, hyaline layer [GO:0033166], egg coat [GO:0035805], cuticular extracellular matrix [GO:0060102], biofilm matrix [GO:0062039], chitin-based extracellular matrix [GO:0062129], pollen coat [GO:0070505], GO:0098965, GO:0099535, GO:1990377 Relationships: is_a extracellular matrix [GO:0031012]